{
  "gene_name": "Actin-related protein 10",
  "gene_symbol": "ACTR10",
  "term_label": "dynactin complex",
  "gene": "UniProtKB:Q9NZ32",
  "term_id": "GO:0005869"
}